{
  "gene": "UniProtKB:P47902",
  "term_id": "GO:0048565",
  "gene_symbol": "CDX1",
  "gene_name": "Homeobox protein CDX-1",
  "term_label": "digestive tract development"
}